D-alanine-alanyl-poly(glycerolphosphate) ligase activity [GO:0047481] (molecular function) Also known as: D-alanine-membrane acceptor-ligase activity, D-alanine:alanyl-poly(glycerolphosphate) ligase (ADP-forming), D-alanine:membrane-acceptor ligase activity, D-alanyl-alanyl-poly(glycerolphosphate) synthetase activity, D-alanyl-poly(phosphoglycerol) synthetase activity, D-alanylalanylpoly(phosphoglycerol) synthetase activity Sources: EC:6.3.2.16, MetaCyc:6.3.2.16-RXN Definition: Catalysis of the reaction: alanyl-poly(glycerolphosphate) + D-alanine + ATP = D-alanyl-alanyl-poly(glycerolphosphate) + phosphate + ADP. Relationships: is a type of acid-amino acid ligase activity [GO:0016881]